{
  "term_id": "UNKNOWN:0003",
  "gene_name": "RNA-binding protein MEX3B",
  "gene_symbol": "MEX3B",
  "gene": "UniProtKB:Q6ZN04",
  "term_label": "Unknown cellular component"
}